{
  "gene_name": "HLA class II histocompatibility antigen gamma chain",
  "gene": "UniProtKB:P04233",
  "term_id": "GO:0070374",
  "term_label": "positive regulation of ERK1 and ERK2 cascade",
  "gene_symbol": "CD74"
}